{
  "gene_name": "Ubiquinol-cytochrome-c reductase complex assembly factor 4",
  "term_label": "Unknown molecular function",
  "term_id": "UNKNOWN:0001",
  "gene_symbol": "UQCC4",
  "gene": "UniProtKB:Q4G0I0"
}